methylglutamate dehydrogenase activity [GO:0050099] (molecular function) Also known as: N-methyl-L-glutamate:(acceptor) oxidoreductase (demethylating), N-methyl-L-glutamate:acceptor oxidoreductase (demethylating), N-methylglutamate dehydrogenase activity Definition: Catalysis of the reaction: N-methyl-L-glutamate + A + H2O = L-glutamate + AH(2) + formaldehyde. Sources: EC:1.5.99.5, RHEA:22572 Relationships: is a type of oxidoreductase activity, acting on the CH-NH group of donors [GO:0016645]